ammonium excretion [GO:0140734] (biological process) Also known as: ammonia excretion References: PMID:25740900 Definition: The elimination of ammonium ions from an excretory cell. Relationships: is a type of excretion [GO:0007588]